{
  "gene_symbol": "MYLK3",
  "term_id": "GO:0045214",
  "term_label": "sarcomere organization",
  "gene": "UniProtKB:Q32MK0",
  "gene_name": "Myosin light chain kinase 3"
}